{
  "gene_name": "Cyclin-G1",
  "term_id": "GO:0016538",
  "gene": "UniProtKB:P51959",
  "gene_symbol": "CCNG1",
  "term_label": "cyclin-dependent protein serine/threonine kinase regulator activity"
}